{
  "term_label": "Unknown cellular component",
  "gene": "UniProtKB:Q8NG35",
  "gene_symbol": "DEFB105B",
  "term_id": "UNKNOWN:0003",
  "gene_name": "Beta-defensin 105"
}